{
  "gene_name": "Alpha-1-syntrophin",
  "term_id": "GO:0031594",
  "term_label": "neuromuscular junction",
  "gene": "UniProtKB:Q13424",
  "gene_symbol": "SNTA1"
}